{
  "gene_name": "Spermatogenesis-associated protein 31A3",
  "gene_symbol": "SPATA31A3",
  "term_id": "UNKNOWN:0002",
  "term_label": "Unknown biological process",
  "gene": "UniProtKB:Q5VYP0"
}